thiamine-containing compound biosynthetic process [GO:0042724] (BP) Also known as: thiamin and derivative biosynthesis, thiamin and derivative biosynthetic process, thiamin-containing compound biosynthetic process, thiamine and derivative biosynthesis, thiamine and derivative biosynthetic process, thiamine-containing compound anabolism, thiamine-containing compound biosynthesis, thiamine-containing compound formation, thiamine-containing compound synthesis, vitamin B1 and derivative biosynthesis, vitamin B1 and derivative biosynthetic process Relationships: is a type of water-soluble vitamin biosynthetic process [GO:0042364]; is a type of GO:0042723; is a type of sulfur compound biosynthetic process [GO:0044272]; is a type of pyrimidine-containing compound biosynthetic process [GO:0072528] Definition: The chemical reactions and pathways resulting in the formation of thiamine (vitamin B1), and related compounds. Subtypes: GO:0009228, thiamine diphosphate biosynthetic process [GO:0009229] Sources: GOC:jl